{
  "gene_name": "EH domain-binding protein 1",
  "gene_symbol": "EHBP1",
  "term_id": "GO:0032456",
  "gene": "UniProtKB:Q8NDI1",
  "term_label": "endocytic recycling"
}